{
  "gene_symbol": "CNTNAP1",
  "gene_name": "Contactin-associated protein 1",
  "gene": "UniProtKB:P78357",
  "term_label": "Unknown molecular function",
  "term_id": "UNKNOWN:0001"
}